{
  "gene_symbol": "LIX1L",
  "term_label": "cytoplasm",
  "gene": "UniProtKB:Q8IVB5",
  "gene_name": "LIX1-like protein",
  "term_id": "GO:0005737"
}